{
  "gene_symbol": "SLURP1",
  "term_label": "acetylcholine receptor activator activity",
  "gene_name": "Secreted Ly-6_uPAR-related protein 1",
  "term_id": "GO:0030549",
  "gene": "UniProtKB:P55000"
}